lectin-induced modified bacterial internalization [GO:0106136] (BP) Relationships: is a type of biological process involved in interaction with symbiont [GO:0051702] Also known as: LIMBI References: PMID:30049880 Sources: GOC:rjd Definition: The process in which an organism effects a change in the structure or function of a symbiont organism, mediated by secretion of lectins which bind to the bacterial surface. The symbiont is defined as the smaller of the organisms involved in a symbiotic interaction.